3'-5' RNA polymerase activity [GO:0097748] (MF) Relationships: is a type of RNA polymerase activity [GO:0097747] Definition: Catalysis of the reaction: nucleoside triphosphate + RNA(n) = diphosphate + RNA(n+1); the synthesis of RNA from ribonucleotide triphosphates in the presence of a nucleic acid template, via extension of the 5'-end. References: PMID:22456265, PMID:27484477, PMID:30917604 Sources: GOC:pf